inositol monophosphate 1-phosphatase activity [GO:0008934] (molecular function) Definition: Catalysis of the reaction: 1D-myo-inositol 1-phosphate + H2O = myo-inositol + phosphate. Relationships: is_a inositol monophosphate phosphatase activity [GO:0052834] Sources: RHEA:27670 Also known as: inositol-1(or 4)-monophosphatase activity, myo-inositol-1(or 4)-monophosphatase activity, myo-inositol-1(or 4)-phosphate phosphohydrolase activity, L-myo-inositol-1-phosphate phosphatase activity, inositol 1-phosphatase activity, myo-inositol 1-phosphatase activity, myo-inositol-1-phosphatase activity